{
  "gene": "UniProtKB:Q12809",
  "term_label": "potassium ion transmembrane transport",
  "gene_name": "Potassium voltage-gated channel subfamily H member 2",
  "term_id": "GO:0071805",
  "gene_symbol": "KCNH2"
}